{
  "gene": "UniProtKB:Q6ZTI0",
  "term_id": "UNKNOWN:0001",
  "term_label": "Unknown molecular function",
  "gene_symbol": "Q6ZTI0",
  "gene_name": "Putative uncharacterized protein FLJ44636"
}